{
  "term_id": "GO:0006995",
  "gene": "UniProtKB:Q9BXW4",
  "gene_name": "Microtubule-associated proteins 1A_1B light chain 3C",
  "term_label": "cellular response to nitrogen starvation",
  "gene_symbol": "MAP1LC3C"
}